Cajal body [GO:0015030] (cellular component) References: PMID:10944589, PMID:11031238, PMID:7559785 Sources: NIF_Subcellular:nlx_subcell_090901 Relationships: is_a nuclear ribonucleoprotein granule [GO:0140168] Also known as: coiled body, Gemini of coiled bodies, Gems Definition: A class of nuclear body, first seen after silver staining by Ramon y Cajal in 1903, enriched in small nuclear ribonucleoproteins, and certain general RNA polymerase II transcription factors; ultrastructurally, they appear as a tangle of coiled, electron-dense threads roughly 0.5 micrometers in diameter; involved in aspects of snRNP biogenesis; the protein coilin serves as a marker for Cajal bodies. Some argue that Cajal bodies are the sites for preassembly of transcriptosomes, unitary particles involved in transcription and processing of RNA.